tolerance induction to nonself antigen [GO:0002462] (biological process) Subtypes: mucosal tolerance induction [GO:0002427], central tolerance induction to nonself antigen [GO:0002463], peripheral tolerance induction to nonself antigen [GO:0002464] Sources: GOC:jal, GO_REF:0000022, ISBN:0781735149 Relationships: is a type of tolerance induction dependent upon immune response [GO:0002461] Definition: Tolerance induction in response to nonself antigens. Regulation: regulated by regulation of tolerance induction to nonself antigen [GO:0002655]; negatively regulated by negative regulation of tolerance induction to nonself antigen [GO:0002656]; positively regulated by positive regulation of tolerance induction to nonself antigen [GO:0002657]